{
  "gene_symbol": "DMRT3",
  "term_label": "RNA polymerase II cis-regulatory region sequence-specific DNA binding",
  "term_id": "GO:0000978",
  "gene": "UniProtKB:Q9NQL9",
  "gene_name": "Doublesex- and mab-3-related transcription factor 3"
}